{
  "gene_name": "Cytochrome c oxidase assembly protein COX19",
  "term_id": "GO:0005758",
  "term_label": "mitochondrial intermembrane space",
  "gene_symbol": "COX19",
  "gene": "UniProtKB:Q49B96"
}